forebrain regionalization [GO:0021871] (biological process) Relationships: is_a regionalization [GO:0003002]; is part of forebrain development [GO:0030900] References: PMID:16226447 Sources: GOC:cls, GOC:dgh, GOC:dph, GOC:isa_complete, GOC:jid Definition: The regionalization process resulting in the creation of areas within the forebrain that will direct the behavior of cell migration in differentiation as the forebrain develops.